antibacterial peptide production [GO:0002778] (BP) References: PMID:11807545, PMID:15638771 Sources: GOC:add, ISBN:0781735149 Relationships: is a type of GO:0002775; is part of antibacterial humoral response [GO:0019731] Note: Note that this term is in the subset of terms that should not be used for direct gene product annotation. Instead, select one of the 'regulation' children terms. Regulation: RO_0002211 by regulation of antibacterial peptide production [GO:0002786]; negatively regulated by negative regulation of antibacterial peptide production [GO:0002787]; RO_0002213 by positive regulation of antibacterial peptide production [GO:0002803] Definition: The synthesis or release of an antibacterial peptide during an immune response, resulting in an increase in intracellular or extracellular levels.